threonine synthase activity [GO:0004795] (molecular function) Definition: Catalysis of the reaction: O-phospho-L-homoserine + H2O = L-threonine + phosphate. Sources: EC:4.2.3.1 Also known as: O-phospho-L-homoserine phospho-lyase (adding water), O-phospho-L-homoserine phospho-lyase (adding water; L-threonine-forming), threonine synthetase activity Relationships: is a type of carbon-oxygen lyase activity, acting on phosphates [GO:0016838]